{
  "gene_symbol": "GLT6D1",
  "term_label": "Unknown biological process",
  "gene": "UniProtKB:Q7Z4J2",
  "gene_name": "Putative glycosyltransferase 6 domain-containing protein 1",
  "term_id": "UNKNOWN:0002"
}